{
  "gene": "UniProtKB:O95049",
  "term_label": "plasma membrane",
  "gene_name": "Tight junction protein ZO-3",
  "term_id": "GO:0005886",
  "gene_symbol": "TJP3"
}